{
  "term_id": "UNKNOWN:0001",
  "gene_name": "Ankyrin repeat and death domain-containing protein 1B",
  "term_label": "Unknown molecular function",
  "gene": "UniProtKB:A6NHY2",
  "gene_symbol": "ANKDD1B"
}